{
  "term_id": "GO:0015871",
  "gene": "UniProtKB:Q8WWI5",
  "gene_symbol": "SLC44A1",
  "term_label": "choline transport",
  "gene_name": "Choline transporter-like protein 1"
}